{
  "gene_name": "Putative uncharacterized protein FLJ43185",
  "term_id": "UNKNOWN:0002",
  "gene": "UniProtKB:P0C879",
  "gene_symbol": "P0C879",
  "term_label": "Unknown biological process"
}